{
  "term_label": "ERAD pathway",
  "gene": "UniProtKB:O00237",
  "gene_symbol": "RNF103",
  "gene_name": "E3 ubiquitin-protein ligase RNF103",
  "term_id": "GO:0036503"
}